{
  "gene": "UniProtKB:Q9NRU3",
  "term_label": "magnesium ion homeostasis",
  "gene_name": "Metal transporter CNNM1",
  "term_id": "GO:0010960",
  "gene_symbol": "CNNM1"
}